branched-chain amino acid catabolic process [GO:0009083] (BP) Definition: The chemical reactions and pathways resulting in the breakdown of amino acids containing a branched carbon skeleton, comprising isoleucine, leucine and valine. Subtypes: branched-chain amino acid catabolic process to alcohol via Ehrlich pathway [GO:0000950], GO:0000953, L-isoleucine catabolic process [GO:0006550], GO:0006552, L-valine catabolic process [GO:0006574], D-leucine catabolic process [GO:1900832], GO:1902079 Also known as: branched chain family amino acid breakdown, branched chain family amino acid catabolic process, branched chain family amino acid catabolism, branched chain family amino acid degradation Sources: GOC:ai Relationships: is a type of GO:0009063; is a type of GO:0009081; is a type of carboxylic acid catabolic process [GO:0046395]